{
  "term_id": "GO:0016251",
  "gene_symbol": "TBPL2",
  "term_label": "RNA polymerase II general transcription initiation factor activity",
  "gene": "UniProtKB:Q6SJ96",
  "gene_name": "TATA box-binding protein-like 2"
}